MIB complex [GO:0140275] (cellular component) Also known as: mitochondrial intermembrane space bridging complex, mitofilin complex Definition: A mitochondrial intermembrane space bridging complex consisting of components of the MICOS complex in the inner mitochondrial membrane, the SAM complex in the outer membrane, a conserved DNAJ protein (human DNAJC11) and Metaxin 1. Relationships: is a type of inner mitochondrial membrane protein complex [GO:0098800] References: PMID:26477565